{
  "term_id": "GO:0005911",
  "gene_name": "V-set and immunoglobulin domain-containing protein 10",
  "term_label": "cell-cell junction",
  "gene": "UniProtKB:Q8N0Z9",
  "gene_symbol": "VSIG10"
}